{
  "gene_symbol": "IGHG2",
  "gene": "UniProtKB:P01859",
  "term_label": "antigen binding",
  "gene_name": "Immunoglobulin heavy constant gamma 2",
  "term_id": "GO:0003823"
}